naphtho-gamma-pyrone biosynthetic process [GO:1900787] (biological process) Relationships: is a type of GO:0042181 Regulation: regulated by GO:1900846; negatively regulated by negative regulation of naphtho-gamma-pyrone biosynthetic process [GO:1900847]; positively regulated by positive regulation of naphtho-gamma-pyrone biosynthetic process [GO:1900848] Subtypes: GO:1900769 Sources: GOC:TermGenie, GOC:di Also known as: naphtho-gamma-pyrone anabolism, naphtho-gamma-pyrone biosynthesis, naphtho-gamma-pyrone formation, naphtho-gamma-pyrone synthesis, naphtho-gamma-pyrones anabolism, naphtho-gamma-pyrones biosynthesis, naphtho-gamma-pyrones biosynthetic process, naphtho-gamma-pyrones formation, naphtho-gamma-pyrones synthesis Definition: The chemical reactions and pathways resulting in the formation of naphtho-gamma-pyrone.